{
  "term_id": "UNKNOWN:0001",
  "term_label": "Unknown molecular function",
  "gene": "UniProtKB:Q15404",
  "gene_name": "Ras suppressor protein 1",
  "gene_symbol": "RSU1"
}